9-cis-epoxycarotenoid dioxygenase activity [GO:0045549] (molecular function) Relationships: is_a carotenoid dioxygenase activity [GO:0010436] Definition: Catalysis of the reactions: a 9-cis-epoxycarotenoid + O2 = 2-cis,4-trans-xanthoxin + a 12'-apo-carotenal; 9-cis-violaxanthin + O2 = 2-cis,4-trans-xanthoxin + (3S,5R,6S)-5,6-epoxy-3-hydroxy-5,6-dihydro-12'-apo-beta-caroten-12'-al; and 9'-cis-neoxanthin + O2 = 2-cis,4-trans-xanthoxin + (3S,5R,6R)-5,6-dihydroxy-6,7-didehydro-5,6-dihydro-12'-apo-beta-caroten-12'-al. Sources: EC:1.13.11.51 Also known as: 9-cis-epoxycarotenoid 11,12-dioxygenase activity, AtNCED3, NCED, PvNCED1, VP14, neoxanthin cleavage enzyme, nine-cis-epoxycarotenoid dioxygenase activity